{
  "gene_name": "Retrotransposon Gag-like protein 6",
  "term_label": "Unknown biological process",
  "term_id": "UNKNOWN:0002",
  "gene": "UniProtKB:Q6ICC9",
  "gene_symbol": "RTL6"
}